{
  "gene_name": "Transmembrane protein 79",
  "term_label": "regulated exocytosis",
  "term_id": "GO:0045055",
  "gene": "UniProtKB:Q9BSE2",
  "gene_symbol": "TMEM79"
}